endocardial cushion fusion [GO:0003274] (biological process) Definition: The cell-cell adhesion process of mesenchymal cardiac cushion cells that contributes to the process of cushion shaping. Relationships: is a type of cell adhesion involved in heart morphogenesis [GO:0061343]; is a type of cell-cell adhesion [GO:0098609]; is part of endocardial cushion morphogenesis [GO:0003203] Sources: GOC:mtg_heart